{
  "gene_symbol": "MYCBP",
  "gene_name": "c-Myc-binding protein",
  "term_id": "GO:0005634",
  "gene": "UniProtKB:Q99417",
  "term_label": "nucleus"
}